{
  "term_label": "fatty acyl-CoA hydrolase activity",
  "term_id": "GO:0047617",
  "gene": "UniProtKB:P49753",
  "gene_symbol": "ACOT2",
  "gene_name": "Acyl-coenzyme A thioesterase 2, mitochondrial"
}